[isocitrate dehydrogenase (NADP+)] kinase activity [GO:0008772] (molecular function) Relationships: is a type of protein serine kinase activity [GO:0106310] Also known as: ICDH kinase/phosphatase activity, IDH kinase/phosphatase activity, IDHK/P, isocitrate dehydrogenase kinase/phosphatase activity, ATP:isocitrate dehydrogenase (NADP+) phosphotransferase activity, IDH kinase activity, IDH-K/P, isocitrate dehydrogenase (NADP) kinase activity, isocitrate dehydrogenase (NADP+) kinase activity, isocitrate dehydrogenase kinase (phosphorylating) activity, isocitrate dehydrogenase kinase activity Definition: Catalysis of the reaction: ATP + L-seryl-[isocitrate dehydrogenase] = ADP + H+ + O-phospho-L-seryl-[isocitrate dehydrogenase]. Sources: RHEA:43540